{
  "term_label": "voltage-gated sodium channel activity",
  "gene_symbol": "SCN4A",
  "gene_name": "Sodium channel protein type 4 subunit alpha",
  "gene": "UniProtKB:P35499",
  "term_id": "GO:0005248"
}